{
  "term_id": "GO:0030215",
  "gene": "UniProtKB:Q9H3T3",
  "term_label": "semaphorin receptor binding",
  "gene_name": "Semaphorin-6B",
  "gene_symbol": "SEMA6B"
}